{
  "term_label": "endoplasmic reticulum membrane",
  "gene_name": "B-cell receptor-associated protein 31",
  "gene": "UniProtKB:P51572",
  "term_id": "GO:0005789",
  "gene_symbol": "BCAP31"
}